{
  "gene": "UniProtKB:Q96FV3",
  "term_id": "UNKNOWN:0001",
  "gene_name": "Tetraspanin-17",
  "gene_symbol": "TSPAN17",
  "term_label": "Unknown molecular function"
}